{
  "gene": "UniProtKB:P25311",
  "gene_symbol": "AZGP1",
  "term_label": "positive regulation of T cell mediated cytotoxicity",
  "term_id": "GO:0001916",
  "gene_name": "Zinc-alpha-2-glycoprotein"
}